regulation of developmental pigmentation [GO:0048070] (biological process) Subtypes: regulation of eye pigmentation [GO:0048073], regulation of cuticle pigmentation [GO:0048079], negative regulation of developmental pigmentation [GO:0048086], GO:0048087, regulation of male pigmentation [GO:0048088], regulation of female pigmentation [GO:0048089] Sources: GOC:dph, GOC:jid, GOC:tb Relationships: is a type of regulation of pigmentation [GO:0120305]; regulates developmental pigmentation [GO:0048066] Also known as: regulation of pigmentation during development Definition: Any process that modulates the frequency, rate or extent of the developmental process that results in the deposition of coloring matter in an organism.